{
  "gene_symbol": "LIN54",
  "term_id": "UNKNOWN:0001",
  "gene_name": "Protein lin-54 homolog",
  "term_label": "Unknown molecular function",
  "gene": "UniProtKB:Q6MZP7"
}